{
  "gene": "UniProtKB:O00175",
  "gene_symbol": "CCL24",
  "term_label": "CCR chemokine receptor binding",
  "term_id": "GO:0048020",
  "gene_name": "C-C motif chemokine 24"
}